nucleolus [GO:0005730] (cellular component) Definition: A small, dense body one or more of which are present in the nucleus of eukaryotic cells. It is rich in RNA and protein, is not bounded by a limiting membrane, and is not seen during mitosis. Its prime function is the transcription of the nucleolar DNA into 45S ribosomal-precursor RNA, the processing of this RNA into 5.8S, 18S, and 28S components of ribosomal RNA, and the association of these components with 5S RNA and proteins synthesized outside the nucleolus. This association results in the formation of ribonucleoprotein precursors; these pass into the cytoplasm and mature into the 40S and 60S subunits of the ribosome. Sources: ISBN:0198506732 Relationships: is a type of intracellular membraneless organelle [GO:0043232]; is part of nuclear lumen [GO:0031981]